{
  "term_id": "UNKNOWN:0001",
  "gene_symbol": "KRTAP9-7",
  "gene_name": "Keratin-associated protein 9-7",
  "gene": "UniProtKB:A8MTY7",
  "term_label": "Unknown molecular function"
}